{
  "gene_symbol": "ZBTB14",
  "term_id": "GO:0000122",
  "gene_name": "Zinc finger and BTB domain-containing protein 14",
  "term_label": "negative regulation of transcription by RNA polymerase II",
  "gene": "UniProtKB:O43829"
}